intestinal epithelial cell migration [GO:0061582] (biological process) Subtypes: colon epithelial cell migration [GO:0061580] Relationships: is a type of epithelial cell migration [GO:0010631] Sources: GOC:dph Definition: The orderly movement of an intestinal epithelial cell from one site to another, often during the development of a multicellular organism.